{
  "gene_name": "Spindle and kinetochore-associated protein 2",
  "term_id": "GO:0007059",
  "gene": "UniProtKB:Q8WVK7",
  "term_label": "chromosome segregation",
  "gene_symbol": "SKA2"
}